{
  "term_id": "GO:0005654",
  "gene": "UniProtKB:Q14978",
  "gene_name": "Nucleolar and coiled-body phosphoprotein 1",
  "term_label": "nucleoplasm",
  "gene_symbol": "NOLC1"
}